{
  "term_id": "GO:1904315",
  "gene_name": "Glutamate receptor ionotropic, kainate 2",
  "term_label": "transmitter-gated monoatomic ion channel activity involved in regulation of postsynaptic membrane potential",
  "gene_symbol": "GRIK2",
  "gene": "UniProtKB:Q13002"
}